{
  "gene_symbol": "PIK3C3",
  "gene": "UniProtKB:Q8NEB9",
  "term_id": "GO:0000045",
  "gene_name": "Phosphatidylinositol 3-kinase catalytic subunit type 3",
  "term_label": "autophagosome assembly"
}